protein lipidation involved in autophagosome assembly [GO:0061739] (biological process) References: PMID:11096062, PMID:11100732, PMID:15277523 Sources: GOC:autophagy, GOC:dph Relationships: is a type of GO:0006501; is part of autophagosome assembly [GO:0000045]; has part Atg8-family ligase activity [GO:0019776]; has part GO:0019779 Definition: The protein lipidation process by which phosphatidylethanolamine is conjugated to a protein of the ATG8 family, leading to membrane insertion of the protein as a step in autophagosome assembly.